{
  "gene": "UniProtKB:Q13324",
  "gene_name": "Corticotropin-releasing factor receptor 2",
  "term_id": "GO:0015056",
  "term_label": "corticotrophin-releasing factor receptor activity",
  "gene_symbol": "CRHR2"
}